regulation of histidine biosynthetic process [GO:0120213] (biological process) Definition: Any process that modulates the frequency, rate or extent of histidine biosynthetic process. Sources: GOC:krc Also known as: regulation of histidine anabolism, regulation of histidine biosynthesis, regulation of histidine formation, regulation of histidine synthesis Relationships: is a type of regulation of small molecule metabolic process [GO:0062012]; is a type of regulation of amino acid biosynthetic process [GO:2000282]; regulates L-histidine biosynthetic process [GO:0000105] Subtypes: negative regulation of histidine biosynthetic process [GO:0120214], positive regulation of histidine biosynthetic process [GO:0120215]